{
  "term_id": "GO:0003712",
  "gene": "UniProtKB:P35637",
  "gene_name": "RNA-binding protein FUS",
  "term_label": "transcription coregulator activity",
  "gene_symbol": "FUS"
}